sucrose alpha-glucosidase activity [GO:0004575] (molecular function) Sources: RHEA:33795 Relationships: is a type of beta-fructofuranosidase activity [GO:0004564]; is a type of alpha-glucosidase activity [GO:0090599] Definition: Catalysis of the reaction: sucrose + H2O = alpha-D-glucose + beta-D-fructose. Also known as: alpha-D-glucopyranosyl beta-D-fructofuranoside hydrolysis, beta-D-fructofuranosyl alpha-D-glucopyranoside hydrolysis, sucrose hydrolysis, sucrose alpha-D-glucohydrolase activity, intestinal sucrase activity, sucrase activity, sucrase(invertase), sucrase-isomaltase activity, sucrose alpha-glucohydrolase activity, sucrose-alpha-D-glucohydrolase activity